prostanoid catabolic process [GO:0062232] (biological process) Relationships: is a type of icosanoid catabolic process [GO:1901523] References: PMID:25449649 Definition: The chemical reactions and pathways resulting in the breakdown of prostanoids. Subtypes: prostaglandin catabolic process [GO:1905344]